diorcinol metabolic process [GO:1900570] (biological process) Sources: GOC:TermGenie, GOC:di Definition: The chemical reactions and pathways involving diorcinol. Subtypes: GO:1900571, diorcinol biosynthetic process [GO:1900572] Relationships: is a type of phenol-containing compound metabolic process [GO:0018958]; is a type of GO:0019748 Also known as: diorcinol metabolism